{
  "term_id": "UNKNOWN:0003",
  "term_label": "Unknown cellular component",
  "gene_name": "N-myc proto-oncogene protein",
  "gene_symbol": "MYCN",
  "gene": "UniProtKB:P04198"
}